template for synthesis of G-rich strand of telomere DNA activity [GO:0000332] (molecular function) Also known as: telomerase RNA, telomerase, template Relationships: is a type of DNA template activity [GO:0000497]; is part of telomerase activity [GO:0003720] References: PMID:11812242, PMID:7958872 Definition: Provision of the template used by reverse transcriptase to synthesize the G-rich strand of telomeric DNA. Note: Note that this term describes the activity of an RNA gene product that interacts with other nucleic acid molecules via base pairing; it should not be used to annotate proteins.